{
  "term_id": "GO:0016126",
  "term_label": "sterol biosynthetic process",
  "gene_name": "3-hydroxy-3-methylglutaryl-coenzyme A reductase",
  "gene_symbol": "HMGCR",
  "gene": "UniProtKB:P04035"
}